{
  "gene_symbol": "CHCHD10",
  "term_id": "GO:0005739",
  "gene_name": "Coiled-coil-helix-coiled-coil-helix domain-containing protein 10, mitochondrial",
  "gene": "UniProtKB:Q8WYQ3",
  "term_label": "mitochondrion"
}